intralumenal vesicle formation [GO:0070676] (biological process) Relationships: is a type of vesicle budding from membrane [GO:0006900]; is a type of GO:0007032; occurs in GO:0010008 References: PMID:19234443 Sources: GOC:jp Definition: The invagination of the endosome membrane and resulting formation of a vesicle within the lumen of the endosome. Also known as: endosome membrane budding Regulation: regulated by regulation of intralumenal vesicle formation [GO:1905365]; negatively regulated by negative regulation of intralumenal vesicle formation [GO:1905366]; positively regulated by GO:1905367